coenzyme gamma-F420-2 biosynthetic process [GO:2001121] (biological process) Also known as: coenzyme gamma-F420-2 biosynthesis Relationships: is a type of alditol phosphate metabolic process [GO:0052646]; is a type of tricarboxylic acid biosynthetic process [GO:0072351]; is a type of GO:0090407; is a type of GO:1901137 Sources: GOC:mengo_curators Definition: The chemical reactions and pathways resulting in the formation of a coenzyme gamma-F420-2.